{
  "gene_symbol": "IL1RN",
  "gene_name": "Interleukin-1 receptor antagonist protein",
  "term_label": "extracellular space",
  "term_id": "GO:0005615",
  "gene": "UniProtKB:P18510"
}